{
  "gene": "UniProtKB:O95678",
  "gene_name": "Keratin, type II cytoskeletal 75",
  "gene_symbol": "KRT75",
  "term_label": "structural constituent of skin epidermis",
  "term_id": "GO:0030280"
}